{
  "gene_symbol": "WDR45B",
  "term_id": "GO:0034045",
  "gene_name": "WD repeat domain phosphoinositide-interacting protein 3",
  "term_label": "phagophore assembly site membrane",
  "gene": "UniProtKB:Q5MNZ6"
}